{
  "gene": "UniProtKB:O94760",
  "gene_symbol": "DDAH1",
  "term_id": "UNKNOWN:0003",
  "gene_name": "N(G),N(G)-dimethylarginine dimethylaminohydrolase 1",
  "term_label": "Unknown cellular component"
}